{
  "gene_symbol": "DDI1",
  "term_label": "regulation of protein stability",
  "gene": "UniProtKB:Q8WTU0",
  "gene_name": "Protein DDI1 homolog 1",
  "term_id": "GO:0031647"
}